{
  "gene": "UniProtKB:Q13536",
  "gene_name": "Protein CROC-4",
  "term_label": "Unknown biological process",
  "gene_symbol": "MIR9-1HG",
  "term_id": "UNKNOWN:0002"
}